positive regulation of pro-T cell differentiation [GO:2000176] (BP) Also known as: positive regulation of pro-T lymphocyte differentiation Relationships: is_a positive regulation of T cell differentiation [GO:0045582]; is_a positive regulation of lymphoid progenitor cell differentiation [GO:1905458]; is a type of GO:2000174; positively regulates GO:0002572 Sources: GOC:BHF Definition: Any process that activates or increases the frequency, rate or extent of pro-T cell differentiation.